{
  "gene_name": "Large ribosomal subunit protein eL6",
  "term_label": "structural constituent of ribosome",
  "gene_symbol": "RPL6",
  "term_id": "GO:0003735",
  "gene": "UniProtKB:Q02878"
}